{
  "term_label": "Unknown biological process",
  "gene": "UniProtKB:P0DMU7",
  "gene_name": "Cancer_testis antigen family 45 member A6",
  "gene_symbol": "CT45A6",
  "term_id": "UNKNOWN:0002"
}